purine ribonucleotide transmembrane transporter activity [GO:0005346] (molecular function) Relationships: is a type of GO:0015216; is a type of carbohydrate derivative transmembrane transporter activity [GO:1901505] Sources: GOC:ai Definition: Enables the transfer of a purine ribonucleotide, any compound consisting of a purine ribonucleoside (a purine organic base attached to a ribose sugar) esterified with (ortho)phosphate, from one side of a membrane to the other. Subtypes: GO:0005347, GTP:GDP antiporter activity [GO:0010292], GO:0015217, 3'-phosphoadenosine 5'-phosphosulfate transmembrane transporter activity [GO:0046964], adenosine 3',5'-bisphosphate transmembrane transporter activity [GO:0071077], GO:0080122, cyclic-GMP-AMP transmembrane transporter activity [GO:0140360], cyclic-di-GMP transmembrane transporter activity [GO:0140927], GO:1902557, ABC-type 3',5'-cyclic GMP transmembrane transporter activity [GO:1905948]